{
  "term_id": "GO:0031466",
  "gene_symbol": "CUL5",
  "gene": "UniProtKB:Q93034",
  "term_label": "Cul5-RING ubiquitin ligase complex",
  "gene_name": "Cullin-5"
}